morphogenesis of an epithelial bud [GO:0060572] (biological process) Subtypes: primary lung bud formation [GO:0060431], prostatic bud formation [GO:0060513], GO:0060648, Malpighian tubule bud morphogenesis [GO:0061332] Sources: GOC:dph Definition: The morphogenetic process in which a bud forms from an epithelial sheet. A bud is a protrusion that forms form the sheet by localized folding. Relationships: is a type of morphogenesis of an epithelial fold [GO:0060571]